{
  "term_label": "cytoplasm",
  "term_id": "GO:0005737",
  "gene_symbol": "CLMN",
  "gene": "UniProtKB:Q96JQ2",
  "gene_name": "Calmin"
}